{
  "term_label": "Unknown biological process",
  "term_id": "UNKNOWN:0002",
  "gene_symbol": "LINC01559",
  "gene": "UniProtKB:Q495D7",
  "gene_name": "Putative uncharacterized protein encoded by LINC01559"
}